{
  "gene_name": "Putative adrenomedullin-5-like protein",
  "gene": "UniProtKB:C9JUS6",
  "gene_symbol": "ADM5",
  "term_id": "GO:0005179",
  "term_label": "hormone activity"
}